{
  "gene": "UniProtKB:Q8WV44",
  "term_id": "GO:0061630",
  "gene_symbol": "TRIM41",
  "gene_name": "E3 ubiquitin-protein ligase TRIM41",
  "term_label": "ubiquitin protein ligase activity"
}